{
  "gene": "UniProtKB:A0A5H1ZRR4",
  "term_id": "UNKNOWN:0001",
  "term_label": "Unknown molecular function",
  "gene_symbol": "TRGJ2",
  "gene_name": "T cell receptor gamma joining 2 (Fragment)"
}